{
  "term_id": "UNKNOWN:0001",
  "gene": "UniProtKB:Q96LR7",
  "gene_name": "Uncharacterized protein C2orf50",
  "term_label": "Unknown molecular function",
  "gene_symbol": "C2orf50"
}